retinal metabolic process [GO:0042574] (biological process) Also known as: retinal metabolism, retinaldehyde metabolic process, retinaldehyde metabolism Relationships: is a type of retinoid metabolic process [GO:0001523]; is a type of aldehyde metabolic process [GO:0006081]; is a type of GO:0120254 Sources: ISBN:0198506732 Definition: The chemical reactions and pathways involving retinal, a compound that plays an important role in the visual process in most vertebrates. In the retina, retinal combines with opsins to form visual pigments. Retinal is one of the forms of vitamin A. Subtypes: retinal isomerization [GO:0106434]